{
  "gene_symbol": "CLRN1",
  "term_id": "GO:0007605",
  "gene_name": "Clarin-1",
  "term_label": "sensory perception of sound",
  "gene": "UniProtKB:P58418"
}